{
  "term_id": "GO:0031410",
  "term_label": "cytoplasmic vesicle",
  "gene_name": "Kinesin-like protein KIF1B",
  "gene_symbol": "KIF1B",
  "gene": "UniProtKB:O60333"
}